{
  "gene_name": "Protein O-mannose kinase",
  "gene": "UniProtKB:Q9H5K3",
  "gene_symbol": "POMK",
  "term_id": "GO:0005789",
  "term_label": "endoplasmic reticulum membrane"
}